{
  "gene": "UniProtKB:Q6NUJ5",
  "gene_name": "PWWP domain-containing protein 2B",
  "gene_symbol": "PWWP2B",
  "term_label": "Unknown molecular function",
  "term_id": "UNKNOWN:0001"
}